{
  "gene": "UniProtKB:Q6ZMV9",
  "term_id": "GO:0005874",
  "gene_name": "Kinesin-like protein KIF6",
  "gene_symbol": "KIF6",
  "term_label": "microtubule"
}